{
  "term_id": "UNKNOWN:0002",
  "gene_name": "Immunoglobulin superfamily member 22",
  "gene_symbol": "IGSF22",
  "gene": "UniProtKB:Q8N9C0",
  "term_label": "Unknown biological process"
}